purine deoxyribonucleoside diphosphate metabolic process [GO:0009182] (biological process) Definition: The chemical reactions and pathways involving purine deoxyribonucleoside diphosphate, a compound consisting of a purine base linked to a deoxyribose sugar esterified with diphosphate on the sugar. Relationships: is a type of purine nucleoside diphosphate metabolic process [GO:0009135] Subtypes: GO:0009183, purine deoxyribonucleoside diphosphate catabolic process [GO:0009184], GO:0046056, dGDP metabolic process [GO:0046066] Sources: GOC:go_curators, ISBN:0198506732 Also known as: purine deoxyribonucleoside diphosphate metabolism